phytanoyl-CoA dioxygenase activity [GO:0048244] (MF) Definition: Catalysis of the reaction: 2-oxoglutarate + O2 + phytanoyl-CoA = 2-hydroxyphytanoyl-CoA + CO2 + succinate. Relationships: is a type of 2-oxoglutarate-dependent dioxygenase activity [GO:0016706] Also known as: phytanoyl-CoA 2 oxoglutarate dioxygenase activity, phytanoyl-CoA 2-hydroxylase activity, phytanoyl-CoA alpha-hydroxylase activity, phytanoyl-CoA hydroxylase activity, phytanoyl-CoA, 2-oxoglutarate:oxygen oxidoreductase (2-hydroxylating) Sources: EC:1.14.11.18, RHEA:16065